{
  "term_id": "GO:0005737",
  "gene_symbol": "DZIP3",
  "gene": "UniProtKB:Q86Y13",
  "term_label": "cytoplasm",
  "gene_name": "E3 ubiquitin-protein ligase DZIP3"
}